{
  "term_label": "fructokinase activity",
  "term_id": "GO:0008865",
  "gene_name": "Hexokinase-4",
  "gene_symbol": "GCK",
  "gene": "UniProtKB:P35557"
}